{
  "gene_symbol": "POLE2",
  "gene_name": "DNA polymerase epsilon subunit 2",
  "term_id": "GO:0006261",
  "term_label": "DNA-templated DNA replication",
  "gene": "UniProtKB:P56282"
}